{
  "term_id": "GO:0098586",
  "term_label": "cellular response to virus",
  "gene": "UniProtKB:Q96DN2",
  "gene_symbol": "VWCE",
  "gene_name": "von Willebrand factor C and EGF domain-containing protein"
}